{
  "term_id": "GO:0005794",
  "gene": "UniProtKB:Q14088",
  "gene_symbol": "RAB33A",
  "term_label": "Golgi apparatus",
  "gene_name": "Ras-related protein Rab-33A"
}